{
  "gene_symbol": "MTPN",
  "term_id": "UNKNOWN:0001",
  "gene_name": "Myotrophin",
  "gene": "UniProtKB:P58546",
  "term_label": "Unknown molecular function"
}